{
  "gene_name": "P antigen family member 1",
  "term_id": "UNKNOWN:0001",
  "term_label": "Unknown molecular function",
  "gene": "UniProtKB:O75459",
  "gene_symbol": "PAGE1"
}